butanediol metabolic process [GO:0034077] (biological process) Subtypes: butanediol catabolic process [GO:0034078], GO:0034079 Definition: The chemical reactions and pathways involving butanediol; the biologically relevant isomer is 2,3-butanediol, CH3CH(OH)CH(OH)CH3. Sources: ISBN:0911910123 Relationships: is_a glycol metabolic process [GO:0042844]; is a type of secondary alcohol metabolic process [GO:1902652] Also known as: butanediol metabolism, butylene glycol metabolic process, butylene glycol metabolism